cellular response to boron-containing substance levels [GO:0080029] (biological process) Also known as: cellular response to boron levels Subtypes: cellular response to boron-containing substance deprivation [GO:0080169] Relationships: is a type of response to boron-containing substance [GO:0010036]; is a type of cellular response to nutrient levels [GO:0031669]; is a type of GO:0070887 References: PMID:18952773 Definition: Any process that results in a change in state or activity of a cell (in terms of movement, secretion, enzyme production, gene expression, etc.) as a result of a stimulus reflecting the presence, absence, or concentration of boron-containing substances.